{
  "term_label": "TAP complex binding",
  "term_id": "GO:0062061",
  "gene": "UniProtKB:Q9BX59",
  "gene_symbol": "TAPBPL",
  "gene_name": "Tapasin-related protein"
}